{
  "term_id": "GO:0005886",
  "term_label": "plasma membrane",
  "gene": "UniProtKB:A8K5M9",
  "gene_name": "Uncharacterized protein C15orf62, mitochondrial",
  "gene_symbol": "C15orf62"
}